{
  "gene_symbol": "GNB2",
  "gene": "UniProtKB:P62879",
  "term_id": "GO:0007186",
  "term_label": "G protein-coupled receptor signaling pathway",
  "gene_name": "Guanine nucleotide-binding protein G(I)_G(S)_G(T) subunit beta-2"
}